{
  "term_id": "GO:0006955",
  "gene": "UniProtKB:A0A075B6S2",
  "term_label": "immune response",
  "gene_symbol": "IGKV2D-29",
  "gene_name": "Immunoglobulin kappa variable 2D-29"
}